{
  "term_label": "dephospho-CoA kinase activity",
  "gene_symbol": "DCAKD",
  "term_id": "GO:0004140",
  "gene": "UniProtKB:Q8WVC6",
  "gene_name": "Dephospho-CoA kinase domain-containing protein"
}